{
  "gene_symbol": "IFI35",
  "gene": "UniProtKB:P80217",
  "term_id": "UNKNOWN:0001",
  "gene_name": "Interferon-induced 35 kDa protein",
  "term_label": "Unknown molecular function"
}